{
  "gene": "UniProtKB:Q9HCC0",
  "gene_symbol": "MCCC2",
  "term_id": "GO:0004485",
  "gene_name": "Methylcrotonoyl-CoA carboxylase beta chain, mitochondrial",
  "term_label": "methylcrotonoyl-CoA carboxylase activity"
}